positive regulation of long-term synaptic depression [GO:1900454] (biological process) Definition: Any process that activates or increases the frequency, rate or extent of long term synaptic depression. Relationships: is_a GO:0048518; is a type of regulation of long-term synaptic depression [GO:1900452]; positively regulates long-term synaptic depression [GO:0060292] Sources: GOC:BHF, GOC:TermGenie Also known as: activation of long term depression, positive regulation of long term depression, up regulation of long term depression, up-regulation of long term depression, upregulation of long term depression, positive regulation of long term synaptic depression, up regulation of long term synaptic depression, up-regulation of long term synaptic depression, upregulation of long term synaptic depression, activation of long term synaptic depression, activation of LTD, positive regulation of LTD, up regulation of LTD, up-regulation of LTD, upregulation of LTD